{
  "gene_symbol": "MED14OS",
  "gene": "UniProtKB:P0DP75",
  "gene_name": "Putative uncharacterized protein MED14OS",
  "term_label": "Unknown biological process",
  "term_id": "UNKNOWN:0002"
}